{
  "gene": "UniProtKB:P21128",
  "gene_symbol": "ENDOU",
  "term_id": "UNKNOWN:0002",
  "gene_name": "Uridylate-specific endoribonuclease",
  "term_label": "Unknown biological process"
}